nucleoside phosphate binding [GO:1901265] (molecular function) Relationships: is a type of binding [GO:0005488] Subtypes: GO:0000166, purine ribonucleoside triphosphate binding [GO:0035639], ADP-D-ribose binding [GO:0072570], coenzyme A binding [GO:0120225], acyl-CoA binding [GO:0120227] Definition: Binding to nucleoside phosphate. Sources: GOC:TermGenie